{
  "term_label": "endoplasmic reticulum",
  "gene_symbol": "P3H1",
  "gene": "UniProtKB:Q32P28",
  "gene_name": "Prolyl 3-hydroxylase 1",
  "term_id": "GO:0005783"
}